{
  "gene": "UniProtKB:P51451",
  "term_label": "cell differentiation",
  "gene_name": "Tyrosine-protein kinase Blk",
  "gene_symbol": "BLK",
  "term_id": "GO:0030154"
}